{
  "gene_symbol": "CT45A5",
  "gene_name": "Cancer_testis antigen family 45 member A5",
  "gene": "UniProtKB:P0DMU8",
  "term_id": "UNKNOWN:0003",
  "term_label": "Unknown cellular component"
}